{
  "gene_name": "Putative golgin subfamily A member 8I",
  "gene": "UniProtKB:A6NC78",
  "term_id": "GO:0007030",
  "term_label": "Golgi organization",
  "gene_symbol": "GOLGA8IP"
}